response to cGMP [GO:0070305] (biological process) Also known as: response to 3',5' cGMP, response to 3',5'-cGMP, response to cyclic GMP, response to guanosine 3',5'-cyclophosphate Sources: GOC:sl Definition: Any process that results in a change in state or activity of a cell or an organism (in terms of movement, secretion, enzyme production, gene expression, etc.) as a result of a cGMP (cyclic GMP, guanosine 3',5'-cyclophosphate) stimulus. Relationships: is a type of response to purine-containing compound [GO:0014074]; is_a response to organophosphorus [GO:0046683]; is a type of response to oxygen-containing compound [GO:1901700] Subtypes: cellular response to cGMP [GO:0071321]